{
  "term_id": "UNKNOWN:0001",
  "gene": "UniProtKB:Q8NDY3",
  "gene_name": "Inactive ADP-ribosyltransferase ARH2",
  "term_label": "Unknown molecular function",
  "gene_symbol": "ADPRHL1"
}